{
  "gene_symbol": "PDGFB",
  "gene_name": "Platelet-derived growth factor subunit B",
  "term_id": "GO:0051897",
  "gene": "UniProtKB:P01127",
  "term_label": "positive regulation of phosphatidylinositol 3-kinase/protein kinase B signal transduction"
}